{
  "term_label": "DNA-binding transcription factor activity, RNA polymerase II-specific",
  "gene_symbol": "RUNX3",
  "gene": "UniProtKB:Q13761",
  "term_id": "GO:0000981",
  "gene_name": "Runt-related transcription factor 3"
}